{
  "gene": "UniProtKB:O94830",
  "gene_symbol": "DDHD2",
  "term_label": "COPII-coated ER to Golgi transport vesicle",
  "gene_name": "Phospholipase DDHD2",
  "term_id": "GO:0030134"
}